{
  "gene": "UniProtKB:P78417",
  "term_label": "glutathione dehydrogenase (ascorbate) activity",
  "term_id": "GO:0045174",
  "gene_name": "Glutathione S-transferase omega-1",
  "gene_symbol": "GSTO1"
}